snRNA methylation [GO:0106349] (biological process) Subtypes: GO:1990437 Definition: The posttranscriptional addition of methyl groups to specific residues in an snRNA molecule. References: PMID:21823225 Relationships: is a type of GO:0001510; is a type of snRNA modification [GO:0040031]